{
  "gene": "UniProtKB:O95452",
  "term_id": "GO:0005922",
  "gene_symbol": "GJB6",
  "gene_name": "Gap junction beta-6 protein",
  "term_label": "connexin complex"
}